{
  "term_label": "cell differentiation",
  "gene_symbol": "NR2F1",
  "term_id": "GO:0030154",
  "gene": "UniProtKB:P10589",
  "gene_name": "COUP transcription factor 1"
}